septum primum development [GO:0003284] (biological process) Definition: The progression of the septum primum over time, from its formation to the mature structure. Sources: GOC:mtg_heart Relationships: is_a atrial septum development [GO:0003283]